negative regulation of axial mesodermal cell fate determination [GO:0048325] (biological process) Definition: Any process that stops, prevents, or reduces the frequency, rate or extent of axial mesoderm cell fate determination. Sources: GOC:dgh Relationships: is a type of GO:0048324; is_a negative regulation of mesodermal cell fate determination [GO:0048335]; negatively regulates axial mesodermal cell fate determination [GO:0048323] Also known as: down regulation of axial mesodermal cell fate determination, down-regulation of axial mesodermal cell fate determination, downregulation of axial mesodermal cell fate determination, inhibition of axial mesodermal cell fate determination